{
  "gene": "UniProtKB:Q9HCG1",
  "term_id": "GO:0000978",
  "gene_name": "Zinc finger protein 160",
  "gene_symbol": "ZNF160",
  "term_label": "RNA polymerase II cis-regulatory region sequence-specific DNA binding"
}